{
  "term_label": "cobalt ion transmembrane transporter activity",
  "gene_name": "Natural resistance-associated macrophage protein 2",
  "gene_symbol": "SLC11A2",
  "gene": "UniProtKB:P49281",
  "term_id": "GO:0015087"
}